transcription factor TFIIH core complex [GO:0000439] (cellular component) References: PMID:14500720, PMID:17215295, PMID:22308316, PMID:22572993, PMID:23028141, PMID:7813015 Sources: GOC:ew, GOC:krc Also known as: SSL2-core TFIIH complex, core TFIIH complex Subtypes: GO:0000438, core TFIIH complex portion of NEF3 complex [GO:0000440] Relationships: is a type of RNA polymerase II transcription regulator complex [GO:0090575] Definition: The 7 subunit core of TFIIH that is a part of either the general transcription factor holo-TFIIH or the nucleotide-excision repair factor 3 complex. In S. cerevisiae/humans the complex is composed of: Ssl2/XPB, Tfb1/p62, Tfb2/p52, Ssl1/p44, Tfb4/p34, Tfb5/p8 and Rad3/XPD.